{
  "term_id": "GO:0004383",
  "gene_symbol": "NPR2",
  "gene": "UniProtKB:P20594",
  "term_label": "guanylate cyclase activity",
  "gene_name": "Atrial natriuretic peptide receptor 2"
}